{
  "gene_name": "Transcription factor 7-like 2",
  "gene_symbol": "TCF7L2",
  "term_id": "GO:0000978",
  "gene": "UniProtKB:Q9NQB0",
  "term_label": "RNA polymerase II cis-regulatory region sequence-specific DNA binding"
}